{
  "gene": "UniProtKB:P50150",
  "gene_name": "Guanine nucleotide-binding protein G(I)_G(S)_G(O) subunit gamma-4",
  "term_id": "GO:0005834",
  "term_label": "heterotrimeric G-protein complex",
  "gene_symbol": "GNG4"
}